{
  "term_id": "UNKNOWN:0001",
  "term_label": "Unknown molecular function",
  "gene": "UniProtKB:Q9NZD4",
  "gene_name": "Alpha-hemoglobin-stabilizing protein",
  "gene_symbol": "AHSP"
}